integrin alpha3-beta1 complex [GO:0034667] (cellular component) Also known as: VLA-3 complex, alpha3-beta1 integrin complex, ITGA3-ITGB1 complex References: PMID:12297042 Relationships: is a type of integrin complex [GO:0008305] Definition: An integrin complex that comprises one alpha3 subunit and one beta1 subunit.